{
  "term_label": "ATPase activator activity",
  "gene": "UniProtKB:P54709",
  "gene_symbol": "ATP1B3",
  "term_id": "GO:0001671",
  "gene_name": "Sodium_potassium-transporting ATPase subunit beta-3"
}